{
  "gene_symbol": "MAPKAPK2",
  "gene_name": "MAP kinase-activated protein kinase 2",
  "term_label": "cellular response to vascular endothelial growth factor stimulus",
  "term_id": "GO:0035924",
  "gene": "UniProtKB:P49137"
}